translational termination [GO:0006415] (biological process) Sources: GOC:hjd, ISBN:019879276X Relationships: is a type of GO:0032984; is part of translation [GO:0006412] Regulation: regulated by GO:0006449; negatively regulated by negative regulation of translational termination [GO:0045904]; positively regulated by positive regulation of translational termination [GO:0045905] Also known as: protein synthesis termination, translation termination, translational complex disassembly Definition: The process resulting in the release of a polypeptide chain from the ribosome, usually in response to a termination codon (UAA, UAG, or UGA in the universal genetic code). Subtypes: cytoplasmic translational termination [GO:0002184], mitochondrial translational termination [GO:0070126]